{
  "gene_name": "Aldehyde dehydrogenase 1A1",
  "gene_symbol": "ALDH1A1",
  "gene": "UniProtKB:P00352",
  "term_id": "GO:0018479",
  "term_label": "benzaldehyde dehydrogenase (NAD+) activity"
}